G protein-coupled bile acid receptor activity [GO:0038182] (molecular function) Also known as: cell surface bile acid receptor, lithocholic acid receptor activity, membrane bile acid receptor activity, G-protein coupled bile acid receptor activity Definition: Combining with an extracellular bile acid and transmitting the signal across the membrane by activating an associated G-protein; promotes the exchange of GDP for GTP on the alpha subunit of a heterotrimeric G-protein complex. References: PMID:12524422, PMID:32480317, PMID:35415765, PMID:36409000 Relationships: is a type of G protein-coupled receptor activity [GO:0004930]; is part of adenylate cyclase-activating G protein-coupled bile acid receptor signaling pathway [GO:0038184]